{
  "term_id": "GO:0070920",
  "gene_name": "RISC-loading complex subunit TARBP2",
  "term_label": "regulation of regulatory ncRNA processing",
  "gene_symbol": "TARBP2",
  "gene": "UniProtKB:Q15633"
}